{
  "gene": "UniProtKB:Q9Y536",
  "term_label": "protein folding",
  "term_id": "GO:0006457",
  "gene_name": "Peptidyl-prolyl cis-trans isomerase A-like 4A",
  "gene_symbol": "PPIAL4A"
}